4-carboxy-2-hydroxymuconate semialdehyde hemiacetal dehydrogenase activity [GO:0050606] (molecular function) Definition: Catalysis of the reaction: 4-carboxy-2-hydroxymuconate semialdehyde hemiacetal + NADP+ = 2-oxo-2H-pyran-4,6-dicarboxylate + H+ + NADPH. Sources: RHEA:29587 Also known as: 2-hydroxy-4-carboxymuconate 6-semialdehyde dehydrogenase activity, 4-carboxy-2-hydroxy-cis,cis-muconate-6-semialdehyde:NADP(+) oxidoreductase activity, 4-carboxy-2-hydroxymuconate-6-semialdehyde dehydrogenase activity, alpha-hydroxy-gamma-carboxymuconic epsilon-semialdehyde dehydrogenase activity Relationships: is a type of GO:0016616